{
  "gene": "UniProtKB:Q8WUU8",
  "gene_name": "Transmembrane protein 174",
  "gene_symbol": "TMEM174",
  "term_id": "UNKNOWN:0003",
  "term_label": "Unknown cellular component"
}